negative regulation of interleukin-35-mediated signaling pathway [GO:0070759] (biological process) Also known as: negative regulation of IL-35-mediated signaling pathway, negative regulation of interleukin-35-mediated signalling pathway Definition: Any process that decreases the rate, frequency or extent of an interleukin-35-mediated signaling pathway. Sources: GOC:mah Relationships: is_a negative regulation of cytokine-mediated signaling pathway [GO:0001960]; is a type of regulation of interleukin-35-mediated signaling pathway [GO:0070758]; negatively regulates GO:0070757